{
  "gene_symbol": "TNXA",
  "term_label": "Unknown cellular component",
  "gene": "UniProtKB:Q16473",
  "term_id": "UNKNOWN:0003",
  "gene_name": "Putative tenascin-XA"
}